{
  "term_id": "UNKNOWN:0001",
  "gene_name": "V-type proton ATPase 16 kDa proteolipid subunit c",
  "gene_symbol": "ATP6V0C",
  "gene": "UniProtKB:P27449",
  "term_label": "Unknown molecular function"
}